{
  "gene_name": "T cell receptor beta variable 10-2",
  "term_label": "cell surface receptor signaling pathway",
  "gene_symbol": "TRBV10-2",
  "gene": "UniProtKB:A0A0K0K1G8",
  "term_id": "GO:0007166"
}